negative regulation of gerfelin biosynthetic process [GO:1900687] (biological process) Relationships: is a type of negative regulation of small molecule metabolic process [GO:0062014]; is a type of negative regulation of secondary metabolite biosynthetic process [GO:1900377]; is_a regulation of gerfelin biosynthetic process [GO:1900686]; negatively regulates gerfelin biosynthetic process [GO:1900578] Also known as: down regulation of gerfelin anabolism, down regulation of gerfelin biosynthesis, down regulation of gerfelin biosynthetic process, down regulation of gerfelin formation, down regulation of gerfelin synthesis, down-regulation of gerfelin anabolism, down-regulation of gerfelin biosynthesis, down-regulation of gerfelin biosynthetic process, down-regulation of gerfelin formation, down-regulation of gerfelin synthesis, downregulation of gerfelin anabolism, downregulation of gerfelin biosynthesis, downregulation of gerfelin biosynthetic process, downregulation of gerfelin formation, downregulation of gerfelin synthesis, inhibition of gerfelin anabolism, inhibition of gerfelin biosynthesis, inhibition of gerfelin formation, inhibition of gerfelin synthesis, negative regulation of gerfelin anabolism, negative regulation of gerfelin biosynthesis, negative regulation of gerfelin formation, negative regulation of gerfelin synthesis, inhibition of gerfelin biosynthetic process Sources: GOC:TermGenie, GOC:di Definition: Any process that stops, prevents or reduces the frequency, rate or extent of gerfelin biosynthetic process.